DNA-DNA tethering activity [GO:0106260] (molecular function) Definition: Bridging together two regions of a DNA molecule. Also known as: double-stranded DNA bridging, dsDNA bridging Subtypes: chromatin loop anchoring activity [GO:0140587] References: PMID:29358048, PMID:30626735 Relationships: is a type of double-stranded DNA binding [GO:0003690]; is a type of molecular adaptor activity [GO:0060090]